alpha-(1->6)-fucosyltransferase activity [GO:0046921] (molecular function) Subtypes: glycoprotein 6-alpha-L-fucosyltransferase activity [GO:0008424], galactoside 6-L-fucosyltransferase activity [GO:0046702] Also known as: alpha(1,6)-fucosyltransferase activity, alpha-(1,6)-fucosyltransferase activity, alpha-1,6-fucosyltransferase activity Sources: GOC:ai Relationships: is a type of GO:0008417 Definition: Catalysis of the transfer of an L-fucosyl group from GDP-beta-L-fucose to an acceptor molecule to form an alpha-(1->6) linkage.